{
  "term_label": "positive regulation of DNA-templated transcription",
  "gene": "UniProtKB:Q9H160",
  "gene_name": "Inhibitor of growth protein 2",
  "term_id": "GO:0045893",
  "gene_symbol": "ING2"
}